{
  "gene_name": "Putative protein FAM47D",
  "gene_symbol": "FAM47DP",
  "gene": "UniProtKB:A6NHR8",
  "term_id": "UNKNOWN:0003",
  "term_label": "Unknown cellular component"
}